{
  "term_label": "fatty acid binding",
  "gene": "UniProtKB:P82980",
  "gene_symbol": "RBP5",
  "gene_name": "Retinol-binding protein 5",
  "term_id": "GO:0005504"
}